protein-disulfide reductase activity [GO:0015035] (molecular function) References: PMID:7559385 Subtypes: flavin-dependent sulfhydryl oxidase activity [GO:0016971], protein-disulfide reductase (glutathione) activity [GO:0019153], protein-disulfide reductase [NAD(P)H] activity [GO:0047134] Definition: Catalysis of the reaction: a protein with reduced sulfide groups = a protein with oxidized disulfide bonds. Also known as: peptide disulfide oxidoreductase activity, peptide disulphide oxidoreductase activity, protein disulfide oxidoreductase activity, protein disulfide-oxidoreductase activity, protein disulphide oxidoreductase activity, haem lyase disulphide oxidoreductase activity, heme lyase disulfide oxidoreductase activity Relationships: is a type of disulfide oxidoreductase activity [GO:0015036]; is a type of catalytic activity, acting on a protein [GO:0140096]